{
  "term_id": "GO:0005615",
  "gene_symbol": "LGALS3BP",
  "term_label": "extracellular space",
  "gene_name": "Galectin-3-binding protein",
  "gene": "UniProtKB:Q08380"
}